{
  "term_id": "GO:0007265",
  "gene_name": "Ras-specific guanine nucleotide-releasing factor 2",
  "gene": "UniProtKB:O14827",
  "term_label": "Ras protein signal transduction",
  "gene_symbol": "RASGRF2"
}